detection of lipopolysaccharide [GO:0032497] (biological process) References: PMID:15998797 Sources: GOC:add Definition: The series of events in which a lipopolysaccharide stimulus is received by a cell and converted into a molecular signal. Lipopolysaccharide is a major component of the cell wall of gram-negative bacteria. Also known as: detection of LPS Relationships: is a type of detection of molecule of bacterial origin [GO:0032490]; is a type of GO:0032496